{
  "gene": "UniProtKB:Q9UQV4",
  "term_id": "GO:0031902",
  "term_label": "late endosome membrane",
  "gene_symbol": "LAMP3",
  "gene_name": "Lysosome-associated membrane glycoprotein 3"
}